{
  "gene_symbol": "TRAF6",
  "gene_name": "TNF receptor-associated factor 6",
  "term_id": "GO:0035591",
  "term_label": "signaling adaptor activity",
  "gene": "UniProtKB:Q9Y4K3"
}